{
  "gene_name": "Paired box protein Pax-6",
  "term_id": "GO:0007420",
  "gene_symbol": "PAX6",
  "term_label": "brain development",
  "gene": "UniProtKB:P26367"
}